{
  "gene": "UniProtKB:P51114",
  "term_label": "positive regulation of translation",
  "term_id": "GO:0045727",
  "gene_symbol": "FXR1",
  "gene_name": "RNA-binding protein FXR1"
}